miRNA transport [GO:1990428] (biological process) Definition: The directed movement of microRNA (miRNA) into, out of or within a cell, or between cells, or within a multicellular organism by means of some agent such as a transporter or pore. Relationships: is a type of RNA transport [GO:0050658] Also known as: microRNA transport References: PMID:24356509 Sources: GO:jl Subtypes: miRNA export from nucleus [GO:0061716]